{
  "term_id": "UNKNOWN:0003",
  "gene_name": "Rho GTPase-activating protein 21",
  "gene_symbol": "ARHGAP21",
  "term_label": "Unknown cellular component",
  "gene": "UniProtKB:Q5T5U3"
}